{
  "gene_name": "Sialic acid-binding Ig-like lectin 14",
  "gene": "UniProtKB:Q08ET2",
  "gene_symbol": "SIGLEC14",
  "term_id": "GO:0007155",
  "term_label": "cell adhesion"
}